sterol O-acyltransferase activity [GO:0004772] (molecular function) Sources: RHEA:59816 Definition: Catalysis of the reaction: a long-chain fatty acyl-CoA + a sterol = a sterol ester + CoA. Subtypes: cholesterol O-acyltransferase activity [GO:0034736], ergosterol O-acyltransferase activity [GO:0034737], lanosterol O-acyltransferase activity [GO:0034738] Relationships: is a type of GO:0008374 Also known as: sterol-ester synthase activity, sterol-ester synthetase activity